negative regulation of ferrichrome biosynthetic process [GO:1905569] (BP) Also known as: down regulation of ferrichrome anabolism, down regulation of ferrichrome biosynthesis, down regulation of ferrichrome biosynthetic process, down regulation of ferrichrome formation, down regulation of ferrichrome synthesis, down-regulation of ferrichrome anabolism, down-regulation of ferrichrome biosynthesis, down-regulation of ferrichrome biosynthetic process, down-regulation of ferrichrome formation, down-regulation of ferrichrome synthesis, downregulation of ferrichrome anabolism, downregulation of ferrichrome biosynthesis, downregulation of ferrichrome biosynthetic process, downregulation of ferrichrome formation, downregulation of ferrichrome synthesis, negative regulation of ferrichrome anabolism, negative regulation of ferrichrome biosynthesis, negative regulation of ferrichrome formation, negative regulation of ferrichrome synthesis, down regulation of ferrichrome biosynthetic process, peptide formation, down regulation of ferrichrome biosynthetic process, peptide modification, down-regulation of ferrichrome biosynthetic process, peptide formation, down-regulation of ferrichrome biosynthetic process, peptide modification, downregulation of ferrichrome biosynthetic process, peptide formation, downregulation of ferrichrome biosynthetic process, peptide modification, inhibition of ferrichrome anabolism, inhibition of ferrichrome biosynthesis, inhibition of ferrichrome biosynthetic process, inhibition of ferrichrome biosynthetic process, peptide formation, inhibition of ferrichrome biosynthetic process, peptide modification, inhibition of ferrichrome formation, inhibition of ferrichrome synthesis, negative regulation of ferrichrome biosynthetic process, peptide formation, negative regulation of ferrichrome biosynthetic process, peptide modification Relationships: is a type of negative regulation of amide metabolic process [GO:0034249]; is a type of negative regulation of siderophore biosynthetic process [GO:1900705]; is a type of regulation of ferrichrome biosynthetic process [GO:1905568]; negatively regulates GO:0031169 References: PMID:654321 Sources: GOC:TermGenie, GOC:al, GO_REF:0000058 Subtypes: negative regulation of ferrichrome biosynthetic process in response to iron [GO:0097739], negative regulation of ferricrocin biosynthetic process [GO:1900679] Definition: Any process that stops, prevents or reduces the frequency, rate or extent of ferrichrome biosynthetic process.